{
  "gene_symbol": "KCTD17",
  "gene": "UniProtKB:Q8N5Z5",
  "gene_name": "BTB_POZ domain-containing protein KCTD17",
  "term_label": "positive regulation of cilium assembly",
  "term_id": "GO:0045724"
}